acyl-lipid omega-(9-4) desaturase activity [GO:0102431] (molecular function) Sources: EC:1.14.19.12 Relationships: is a type of monooxygenase activity [GO:0004497]; is a type of oxidoreductase activity, acting on paired donors, with oxidation of a pair of donors resulting in the reduction of molecular oxygen to two molecules of water [GO:0016717] Definition: Catalysis of the reaction: a (9Z,12Z)-octadecadienoyl-containing glycerolipid + 2 Fe(II)-[cytochrome b5] + 2 H+ + O2 = a (5Z,9Z,12Z)-octadecatrienoyl-containing glycerolipid + 2 Fe(III)-[cytochrome b5] + 2 H2O. Can also use a substrate with 3 double bonds (a (9Z,12Z,15Z)-octadecatrienoyl-containing glycerolipid) and add a fourth double bond (a (5Z,9Z,12Z,15Z)-octadecatetraenoyl-containing glycerolipid). Also known as: acyl-lipid omega-(9-4) desaturase, alpha-linolenate delta5 desaturase activity, linoleate delta5 desaturase activity